hepatic duct development [GO:0061011] (biological process) References: PMID:20614624 Sources: GOC:dph Definition: The progression of the hepatic duct over time, from its formation to the mature structure. The hepatic duct is the duct that leads from the liver to the common bile duct. Relationships: is a type of GO:0061009